{
  "gene_symbol": "FZR1",
  "term_id": "GO:0005680",
  "term_label": "anaphase-promoting complex",
  "gene": "UniProtKB:Q9UM11",
  "gene_name": "Fizzy-related protein homolog"
}